{
  "term_label": "Unknown biological process",
  "term_id": "UNKNOWN:0002",
  "gene_symbol": "TIGD2",
  "gene": "UniProtKB:Q4W5G0",
  "gene_name": "Tigger transposable element-derived protein 2"
}